meiotic nuclear membrane reassembly [GO:0051333] (BP) Definition: The cell cycle process in which the reformation of the nuclear membranes during meiosis occurs. Relationships: is a type of GO:0031468; is a type of GO:1903046 Subtypes: meiosis I nuclear membrane reassembly [GO:0051334], meiosis II nuclear membrane reassembly [GO:0051335] Sources: GOC:ai Also known as: meiotic nuclear envelope reassembly